{
  "gene_name": "Endoplasmic reticulum protein SC65",
  "term_label": "endoplasmic reticulum",
  "gene": "UniProtKB:Q92791",
  "term_id": "GO:0005783",
  "gene_symbol": "P3H4"
}